{
  "gene_symbol": "POTEKP",
  "term_label": "synapse",
  "gene": "UniProtKB:Q9BYX7",
  "gene_name": "Putative beta-actin-like protein 3",
  "term_id": "GO:0045202"
}